glial cell differentiation [GO:0010001] (biological process) Relationships: is a type of cell differentiation [GO:0030154]; is part of GO:0042063 Sources: GOC:go_curators, GOC:mtg_sensu Regulation: regulated by GO:0045685; negatively regulated by negative regulation of glial cell differentiation [GO:0045686]; positively regulated by positive regulation of glial cell differentiation [GO:0045687] Definition: The process in which a relatively unspecialized cell acquires the specialized features of a glial cell. Also known as: glia cell differentiation, neuroglia differentiation Subtypes: GO:0003398, microglia differentiation [GO:0014004], GO:0014037, astrocyte differentiation [GO:0048708], oligodendrocyte differentiation [GO:0048709], lateral line nerve glial cell differentiation [GO:0048895], GO:0060019, GO:0060950